{
  "gene_symbol": "IQCH",
  "gene": "UniProtKB:Q86VS3",
  "term_label": "Unknown biological process",
  "term_id": "UNKNOWN:0002",
  "gene_name": "IQ domain-containing protein H"
}